deaminase binding [GO:1990827] (MF) References: PMID:9792439 Relationships: is a type of enzyme binding [GO:0019899] Definition: Binding to an enzyme that catalyzes the removal of an amino group from a substrate, producing ammonia (NH3).